regulation of protein ubiquitination [GO:0031396] (biological process) Relationships: is a type of GO:1903320; RO_0002211 protein ubiquitination [GO:0016567] Definition: Any process that modulates the frequency, rate or extent of the addition of ubiquitin groups to a protein. Sources: GOC:mah Subtypes: negative regulation of protein ubiquitination [GO:0031397], positive regulation of protein ubiquitination [GO:0031398], regulation of protein autoubiquitination [GO:1902498], regulation of protein monoubiquitination [GO:1902525], regulation of protein polyubiquitination [GO:1902914]